{
  "gene": "UniProtKB:A0A075B6S4",
  "gene_symbol": "IGKV1D-17",
  "term_id": "UNKNOWN:0001",
  "term_label": "Unknown molecular function",
  "gene_name": "Immunoglobulin kappa variable 1D-17"
}